2-alkenal reductase (NADPH) activity [GO:0035798] (molecular function) References: PMID:16299173 Sources: RHEA:13737 Also known as: NADPH:2-alkenal alpha,beta-hydrogenase activity Definition: Catalysis of the reaction: n-alkanal + NADP+ = alk-2-enal + NADPH + H+. Relationships: is a type of 2-alkenal reductase [NAD(P)H] activity [GO:0032440]